metanephric juxtaglomerular apparatus development [GO:0072206] (biological process) Relationships: is a type of juxtaglomerular apparatus development [GO:0072051]; is part of GO:0001656 Sources: GOC:mtg_kidney_jan10 Definition: The process whose specific outcome is the progression of the juxtaglomerular apparatus in the metanephros over time, from its formation to the mature structure. The juxtaglomerular apparatus is an anatomical structure which consists of juxtaglomerular cells, extraglomerular mesangial cells and the macula densa. The juxtaglomerular apparatus lies adjacent to the glomerulus and regulates kidney function by maintaining the blood flow to the kidney and the filtration rate.